{
  "gene": "UniProtKB:Q96CQ1",
  "term_id": "GO:0005739",
  "gene_name": "Solute carrier family 25 member 36",
  "gene_symbol": "SLC25A36",
  "term_label": "mitochondrion"
}